{
  "gene_name": "Glutathione S-transferase Mu 5",
  "term_id": "GO:0006749",
  "gene_symbol": "GSTM5",
  "term_label": "glutathione metabolic process",
  "gene": "UniProtKB:P46439"
}